{
  "term_id": "GO:0097729",
  "gene": "UniProtKB:Q8WXX0",
  "gene_name": "Dynein axonemal heavy chain 7",
  "gene_symbol": "DNAH7",
  "term_label": "9+2 motile cilium"
}